{
  "term_label": "endoplasmic reticulum-Golgi intermediate compartment",
  "gene_name": "Protein ERGIC-53-like",
  "gene_symbol": "LMAN1L",
  "gene": "UniProtKB:Q9HAT1",
  "term_id": "GO:0005793"
}